{
  "gene_name": "DNA-directed RNA polymerase I subunit RPA34",
  "term_id": "GO:0005736",
  "gene_symbol": "POLR1G",
  "gene": "UniProtKB:O15446",
  "term_label": "RNA polymerase I complex"
}